interleukin-1, type I receptor binding [GO:0005150] (molecular function) Sources: GOC:ai Relationships: is a type of interleukin-1 receptor binding [GO:0005149] Definition: Binding to a Type I interleukin-1 receptor. Also known as: IL-1 type I, interleukin-1, type I receptor ligand